{
  "term_label": "Unknown cellular component",
  "gene": "UniProtKB:P60369",
  "gene_symbol": "KRTAP10-3",
  "term_id": "UNKNOWN:0003",
  "gene_name": "Keratin-associated protein 10-3"
}